{
  "gene": "UniProtKB:P52429",
  "gene_symbol": "DGKE",
  "gene_name": "Diacylglycerol kinase epsilon",
  "term_id": "GO:0035556",
  "term_label": "intracellular signal transduction"
}